{
  "term_label": "Unknown cellular component",
  "gene": "UniProtKB:Q13278",
  "gene_symbol": "RIG",
  "term_id": "UNKNOWN:0003",
  "gene_name": "Putative protein RIG"
}